{
  "gene_symbol": "TUBA1A",
  "term_id": "GO:0000278",
  "gene_name": "Tubulin alpha-1A chain",
  "term_label": "mitotic cell cycle",
  "gene": "UniProtKB:Q71U36"
}